{
  "gene_name": "Myoglobin",
  "gene_symbol": "MB",
  "term_id": "GO:0016528",
  "term_label": "sarcoplasm",
  "gene": "UniProtKB:P02144"
}